{
  "gene_symbol": "KIF16B",
  "term_label": "kinesin complex",
  "term_id": "GO:0005871",
  "gene_name": "Kinesin-like protein KIF16B",
  "gene": "UniProtKB:Q96L93"
}